{
  "gene_name": "C-C chemokine receptor type 6",
  "term_id": "GO:0016493",
  "term_label": "C-C chemokine receptor activity",
  "gene_symbol": "CCR6",
  "gene": "UniProtKB:P51684"
}